{
  "gene_name": "ATPase SWSAP1",
  "gene_symbol": "SWSAP1",
  "term_id": "GO:0000724",
  "term_label": "double-strand break repair via homologous recombination",
  "gene": "UniProtKB:Q6NVH7"
}